positive regulation of orcinol biosynthetic process [GO:1900703] (biological process) Sources: GOC:TermGenie, GOC:di Also known as: activation of orcinol anabolism, activation of orcinol biosynthesis, activation of orcinol formation, activation of orcinol synthesis, positive regulation of orcinol anabolism, positive regulation of orcinol biosynthesis, positive regulation of orcinol formation, positive regulation of orcinol synthesis, up regulation of orcinol anabolism, up regulation of orcinol biosynthesis, up regulation of orcinol biosynthetic process, up regulation of orcinol formation, up regulation of orcinol synthesis, up-regulation of orcinol anabolism, up-regulation of orcinol biosynthesis, up-regulation of orcinol biosynthetic process, up-regulation of orcinol formation, up-regulation of orcinol synthesis, upregulation of orcinol anabolism, upregulation of orcinol biosynthesis, upregulation of orcinol biosynthetic process, upregulation of orcinol formation, upregulation of orcinol synthesis, activation of orcinol biosynthetic process Definition: Any process that activates or increases the frequency, rate or extent of orcinol biosynthetic process. Relationships: is a type of positive regulation of secondary metabolite biosynthetic process [GO:1900378]; is a type of regulation of orcinol biosynthetic process [GO:1900701]; positively regulates orcinol biosynthetic process [GO:0046197]